{
  "gene": "UniProtKB:O14603",
  "term_label": "Unknown molecular function",
  "gene_symbol": "PRYP4",
  "term_id": "UNKNOWN:0001",
  "gene_name": "PTPN13-like protein, Y-linked"
}